inositol hexakisphosphate phosphatase activity [GO:0004446] (molecular function) Subtypes: inositol hexakisphosphate 4-phosphatase activity [GO:0008707], inositol hexakisphosphate 3-phosphatase activity [GO:0016158], inositol hexakisphosphate 5-phosphatase activity [GO:0050533] Relationships: is a type of inositol phosphate phosphatase activity [GO:0052745] Sources: GOC:curators Definition: Catalysis of the reaction: myo-inositol hexakisphosphate + H2O = myo-inositol pentakisphosphate + phosphate.